{
  "term_id": "UNKNOWN:0001",
  "gene": "UniProtKB:Q7Z7G8",
  "gene_name": "Intermembrane lipid transfer protein VPS13B",
  "gene_symbol": "VPS13B",
  "term_label": "Unknown molecular function"
}